{
  "term_id": "GO:0042470",
  "gene_name": "Ras-related protein Rab-7L1",
  "gene_symbol": "RAB29",
  "gene": "UniProtKB:O14966",
  "term_label": "melanosome"
}